regulation of striated muscle contraction [GO:0006942] (BP) Sources: GOC:go_curators Definition: Any process that modulates the frequency, rate or extent of striated muscle contraction. Subtypes: GO:0014819, negative regulation of striated muscle contraction [GO:0045988], positive regulation of striated muscle contraction [GO:0045989], regulation of cardiac muscle contraction [GO:0055117] Relationships: is a type of regulation of muscle contraction [GO:0006937]; regulates striated muscle contraction [GO:0006941]